{
  "term_id": "UNKNOWN:0002",
  "gene_symbol": "CSTF1",
  "term_label": "Unknown biological process",
  "gene": "UniProtKB:Q05048",
  "gene_name": "Cleavage stimulation factor subunit 1"
}